cholesterol 25-hydroxylase activity [GO:0001567] (molecular function) Definition: Catalysis of the reaction: AH2 + cholesterol + O2 = 25-hydroxycholesterol + A + H2O. Relationships: is a type of steroid hydroxylase activity [GO:0008395]; is a type of oxidoreductase activity, acting on paired donors, with incorporation or reduction of molecular oxygen [GO:0016705] Also known as: cholesterol 25-monooxygenase activity, cholesterol,hydrogen-donor:oxygen oxidoreductase (25-hydroxylating) activity Sources: RHEA:21104